{
  "term_label": "Unknown biological process",
  "gene_name": "Laminin subunit gamma-2",
  "gene_symbol": "LAMC2",
  "term_id": "UNKNOWN:0002",
  "gene": "UniProtKB:Q13753"
}